{
  "gene_symbol": "IFNK",
  "gene_name": "Interferon kappa",
  "term_label": "response to exogenous dsRNA",
  "term_id": "GO:0043330",
  "gene": "UniProtKB:Q9P0W0"
}